medial fin morphogenesis [GO:0035141] (biological process) Sources: GOC:dgh Also known as: median fin morphogenesis, unpaired fin morphogenesis Subtypes: embryonic medial fin morphogenesis [GO:0035122], post-embryonic medial fin morphogenesis [GO:0035132], dorsal fin morphogenesis [GO:0035142], caudal fin morphogenesis [GO:0035143], anal fin morphogenesis [GO:0035144] Definition: The process in which the anatomical structures of the medial fin are generated and organized. A medial fin is an unpaired fin of fish, usually located dorsomedially or ventromedially and primarily used for stability while swimming. Relationships: is a type of fin morphogenesis [GO:0033334]; is part of medial fin development [GO:0033338]